cytosolic ribosome assembly [GO:0042256] (biological process) References: PMID:30467428 Sources: GOC:ma Relationships: is a type of GO:0042255 Also known as: mature ribosome assembly Definition: The aggregation, arrangement and bonding together of the large and small ribosomal subunits into a functional cytosolic ribosome. Distinct stages of this process take place first in the nucleolus, then in the nucleus and finally in the cytosol.